{
  "gene_symbol": "IL22RA2",
  "gene": "UniProtKB:Q969J5",
  "gene_name": "Interleukin-22 receptor subunit alpha-2",
  "term_label": "cytokine receptor activity",
  "term_id": "GO:0004896"
}